{
  "gene": "UniProtKB:Q9H2U9",
  "term_label": "metalloendopeptidase activity",
  "gene_symbol": "ADAM7",
  "gene_name": "Disintegrin and metalloproteinase domain-containing protein 7",
  "term_id": "GO:0004222"
}